{
  "gene": "UniProtKB:Q9BYW1",
  "term_label": "D-glucose transmembrane transporter activity",
  "gene_symbol": "SLC2A11",
  "gene_name": "Solute carrier family 2, facilitated glucose transporter member 11",
  "term_id": "GO:0055056"
}